{
  "gene_symbol": "ZNF639",
  "gene_name": "Zinc finger protein 639",
  "term_id": "UNKNOWN:0003",
  "gene": "UniProtKB:Q9UID6",
  "term_label": "Unknown cellular component"
}